{
  "term_label": "extracellular space",
  "gene": "UniProtKB:P09871",
  "gene_symbol": "C1S",
  "term_id": "GO:0005615",
  "gene_name": "Complement C1s subcomponent"
}